{
  "gene_name": "Dihydrofolate reductase 2, mitochondrial",
  "gene_symbol": "DHFR2",
  "term_label": "dihydrofolate reductase activity",
  "term_id": "GO:0004146",
  "gene": "UniProtKB:Q86XF0"
}